{
  "term_id": "UNKNOWN:0003",
  "gene_symbol": "MRO",
  "gene_name": "Protein maestro",
  "gene": "UniProtKB:Q9BYG7",
  "term_label": "Unknown cellular component"
}